negative regulation of reproductive process [GO:2000242] (biological process) Definition: Any process that stops, prevents, or reduces the frequency, rate or extent of reproductive process. Relationships: is_a GO:0048519; is a type of regulation of reproductive process [GO:2000241]; negatively regulates reproductive process [GO:0022414] Sources: GOC:mah Subtypes: negative regulation of flower development [GO:0009910], negative regulation of meiotic joint molecule formation [GO:0010947], negative regulation of conjugation with cellular fusion [GO:0031138], negative regulation of mating type switching [GO:0031495], negative regulation of fusion of sperm to egg plasma membrane [GO:0043013], GO:0045593, negative regulation of embryo sac egg cell differentiation [GO:0045695], negative regulation of spermatid nuclear differentiation [GO:0045701], negative regulation of nurse cell apoptotic process [GO:0045849], GO:0048090, negative regulation of male pigmentation [GO:0048092], negative regulation of meiotic cell cycle [GO:0051447], GO:0060240, negative regulation of ovulation [GO:0060280], negative regulation of oocyte development [GO:0060283], negative regulation of penile erection [GO:0060407], negative regulation of fertilization [GO:0060467], negative regulation of prostatic bud formation [GO:0060686], GO:0060770, GO:0060806, negative regulation of floral organ abscission [GO:0060862], GO:0061950, negative regulation of conidiophore stalk development [GO:0070800], negative regulation of metula development [GO:0070803], GO:0070809, GO:0075262, negative regulation of anther dehiscence [GO:0120196], negative regulation of oocyte karyosome formation [GO:0120314], negative regulation of oocyte maturation [GO:1900194], negative regulation of egg-laying behavior [GO:1901045], negative regulation of trophoblast cell migration [GO:1901164], negative regulation of flagellated sperm motility [GO:1901318], negative regulation of seed dormancy process [GO:1902039], negative regulation of acrosome reaction [GO:1902225], GO:1902436, negative regulation of sperm capacitation [GO:1902491], negative regulation of meiotic DNA double-strand break formation [GO:1903342], negative regulation of asexual reproduction [GO:1903665], negative regulation of endosperm development [GO:1904095], negative regulation of maternal process involved in parturition [GO:1904302], negative regulation of establishment of Sertoli cell barrier [GO:1904445], negative regulation of meiotic chromosome separation [GO:1905133], GO:1905417, negative regulation of oogenesis [GO:1905880], negative regulation of gonad development [GO:1905940], negative regulation of FtsZ-dependent cytokinesis [GO:2000245], negative regulation of male germ cell proliferation [GO:2000255], negative regulation of binding of sperm to zona pellucida [GO:2000360], negative regulation of seed maturation [GO:2000692]